aspyridone B biosynthetic process [GO:1901521] (biological process) Sources: GOC:TermGenie, GOC:di Also known as: aspyridone B anabolism, aspyridone B biosynthesis, aspyridone B formation, aspyridone B synthesis Definition: The chemical reactions and pathways resulting in the formation of aspyridone B. Relationships: is a type of polyketide biosynthetic process [GO:0030639]; is a type of pyridine-containing compound biosynthetic process [GO:0072525]